{
  "term_label": "Unknown molecular function",
  "gene_symbol": "NPHP3",
  "gene": "UniProtKB:Q7Z494",
  "term_id": "UNKNOWN:0001",
  "gene_name": "Nephrocystin-3"
}